{
  "term_id": "GO:0045944",
  "gene": "UniProtKB:Q9NQV6",
  "gene_name": "PR domain zinc finger protein 10",
  "term_label": "positive regulation of transcription by RNA polymerase II",
  "gene_symbol": "PRDM10"
}